{
  "gene_name": "Caspase-3",
  "term_label": "erythrocyte differentiation",
  "gene_symbol": "CASP3",
  "term_id": "GO:0030218",
  "gene": "UniProtKB:P42574"
}